Ycf2/FtsHi complex [GO:0062091] (cellular component) Also known as: TIC complex associated chloroplast protein import motor Definition: A protein complex located in the chloroplast inner membrane and facing the stroma that is associated with the chloroplast inner membrane translocase complex and provides the ATPase motor activity to drive import of proteins into the chloroplast stroma. Relationships: is a type of GO:1904949 References: PMID:30309901